{
  "gene": "UniProtKB:Q5NDL2",
  "term_label": "Unknown biological process",
  "gene_name": "EGF domain-specific O-linked N-acetylglucosamine transferase",
  "term_id": "UNKNOWN:0002",
  "gene_symbol": "EOGT"
}